endospore external encapsulating structure [GO:0043591] (cellular component) Definition: The structures that lie outside the inner membrane and surround the entire endospore; consists of a peptidoglycan-containing inner layer (the endospore cortex) surrounded by a multilayered proteinaceous coat. An exosporium may be present as an extreme outer layer. References: PMID:15035041 Sources: GOC:go_curators Also known as: spore wall, endospore wall, peptidoglycan-based spore wall Relationships: is a type of spore wall [GO:0031160]